{
  "term_id": "GO:0005546",
  "gene_symbol": "GSDMD",
  "term_label": "phosphatidylinositol-4,5-bisphosphate binding",
  "gene": "UniProtKB:P57764",
  "gene_name": "Gasdermin-D"
}